cellular response to glycoprotein [GO:1904588] (biological process) Definition: Any process that results in a change in state or activity of a cell (in terms of movement, secretion, enzyme production, gene expression, etc.) as a result of a glycoprotein stimulus. References: PMID:14597422 Sources: GOC:TermGenie, GO_REF:0000071 Also known as: cellular response to glycoproteins Relationships: is a type of cellular response to nitrogen compound [GO:1901699]; is a type of cellular response to oxygen-containing compound [GO:1901701]; is a type of GO:1904587 Subtypes: cellular response to Thyroid stimulating hormone [GO:1904401], cellular response to carcinoembryonic antigen [GO:1990831]